{
  "gene_name": "Olfactory receptor 4N4C",
  "term_label": "olfactory receptor activity",
  "gene_symbol": "OR4N4C",
  "term_id": "GO:0004984",
  "gene": "UniProtKB:A0A096LPK9"
}